Pwp2p-containing subcomplex of 90S preribosome [GO:0034388] (CC) References: PMID:15231838 Sources: GOC:krc Also known as: 25-30 S subcomplex of 90S preribosome, UTP-B complex Relationships: is_a nuclear protein-containing complex [GO:0140513]; is part of nucleolus [GO:0005730]; is part of 90S preribosome [GO:0030686] Note: Note that the term name uses Saccharomyces gene product names because no other names have yet arisen for this complex; the term nevertheless can be used for analogous complexes in other eukaryotes, and the name can be changed if better wording is found. Definition: A protein complex that forms a subcomplex of the 90S preribosome and can interact directly with the 5' External Transcribed Spacer (ETS) of the full length pre-rRNA transcript. In S. cerevisiae, it sediments at 25-30 S and is composed of Pwp2p, Dip2p, Utp21p, Utp13p, Utp18p, and Utp6p.